protein-phosphocysteine-N-acetylglucosamine phosphotransferase system transporter activity [GO:0090586] (molecular function) Relationships: is a type of protein-phosphocysteine-sugar phosphotransferase activity [GO:0090563] References: PMID:8246840 Definition: Catalysis of the PEP-dependent, phosphoryl transfer-driven transport of substances across a membrane. The transport happens by catalysis of the reaction: protein S-phosphocysteine + N-acetylglucosamine (out) = protein cysteine + N-acetylglucosamine-6-phosphate (in).